{
  "term_id": "GO:0006357",
  "gene": "UniProtKB:Q8IWS0",
  "gene_symbol": "PHF6",
  "gene_name": "PHD finger protein 6",
  "term_label": "regulation of transcription by RNA polymerase II"
}